{
  "term_id": "UNKNOWN:0003",
  "gene_symbol": "TMC4",
  "term_label": "Unknown cellular component",
  "gene": "UniProtKB:Q7Z404",
  "gene_name": "Transmembrane channel-like protein 4"
}